{
  "gene": "UniProtKB:Q8N0S6",
  "gene_name": "Centromere protein L",
  "term_id": "UNKNOWN:0001",
  "term_label": "Unknown molecular function",
  "gene_symbol": "CENPL"
}